Dsl1/NZR complex [GO:0070939] (cellular component) Note: See also the molecular function term 'acetolactate synthase activity ; GO:0003984'. References: PMID:19151722, PMID:21550981 Sources: GOC:jh, GOC:mah Relationships: is a type of vesicle tethering complex [GO:0099023]; is a type of endoplasmic reticulum protein-containing complex [GO:0140534] Also known as: CATCHR family complex, Dsl1p complex, NZR complex Definition: A multisubunit tethering complex, i.e. a protein complex involved in mediating the initial interaction between vesicles and the membranes with which they fuse, that is involved in trafficking from the Golgi apparatus to the ER. In Saccharomyces cerevisiae the Dsl1p complex contains Dsl1p, Tip20p, and Sec39p.